photosystem II antenna complex [GO:0009783] (cellular component) Definition: The antenna complex of photosystem II. A photosystem has two closely linked components, an antenna containing light-absorbing pigments and a reaction center. Each antenna contains one or more light-harvesting complexes (LHCs). Sources: GOC:jid, ISBN:0716731363 Relationships: is a type of membrane protein complex [GO:0098796]; is part of photosystem II [GO:0009523]